{
  "gene": "UniProtKB:O00764",
  "term_label": "pyridoxal 5'-phosphate salvage",
  "term_id": "GO:0009443",
  "gene_symbol": "PDXK",
  "gene_name": "Pyridoxal kinase"
}